{
  "term_label": "Unknown biological process",
  "term_id": "UNKNOWN:0002",
  "gene": "UniProtKB:Q6P3S6",
  "gene_name": "F-box only protein 42",
  "gene_symbol": "FBXO42"
}